{
  "term_label": "MHC class II protein complex binding",
  "gene_symbol": "HLA-DRB4",
  "gene_name": "HLA class II histocompatibility antigen, DR beta 4 chain",
  "term_id": "GO:0023026",
  "gene": "UniProtKB:P13762"
}